{
  "gene_symbol": "ATF6B",
  "term_label": "endoplasmic reticulum unfolded protein response",
  "gene": "UniProtKB:Q99941",
  "gene_name": "Cyclic AMP-dependent transcription factor ATF-6 beta",
  "term_id": "GO:0030968"
}